{
  "gene_symbol": "GPR141",
  "gene_name": "Probable G-protein coupled receptor 141",
  "term_label": "Unknown cellular component",
  "term_id": "UNKNOWN:0003",
  "gene": "UniProtKB:Q7Z602"
}